RNA-templated DNA biosynthetic process [GO:0006278] (BP) Sources: GOC:mah, ISBN:0198506732 Subtypes: GO:0001171, telomere maintenance via telomerase [GO:0007004] Relationships: is a type of DNA biosynthetic process [GO:0071897] Definition: A DNA biosynthetic process that uses RNA as a template for RNA-dependent DNA polymerases (e.g. reverse transcriptase) that synthesize the new strand. Also known as: RNA-dependent DNA biosynthetic process